{
  "gene": "UniProtKB:Q9H322",
  "term_label": "Unknown molecular function",
  "gene_symbol": "VCX2",
  "gene_name": "Variable charge X-linked protein 2",
  "term_id": "UNKNOWN:0001"
}